{
  "gene": "UniProtKB:Q5TD94",
  "term_id": "UNKNOWN:0001",
  "gene_symbol": "RSPH4A",
  "term_label": "Unknown molecular function",
  "gene_name": "Radial spoke head protein 4 homolog A"
}